{
  "gene": "UniProtKB:A0A5B6",
  "term_label": "plasma membrane",
  "gene_symbol": "TRBV28",
  "gene_name": "T cell receptor beta variable 28",
  "term_id": "GO:0005886"
}